positive regulation of eosinophil chemotaxis [GO:2000424] (biological process) Sources: GOC:obol Relationships: is a type of positive regulation of granulocyte chemotaxis [GO:0071624]; is a type of positive regulation of eosinophil migration [GO:2000418]; is a type of regulation of eosinophil chemotaxis [GO:2000422]; positively regulates eosinophil chemotaxis [GO:0048245] Definition: Any process that activates or increases the frequency, rate or extent of eosinophil chemotaxis.